{
  "term_label": "plasma membrane",
  "gene_symbol": "TAAR5",
  "gene_name": "Trace amine-associated receptor 5",
  "gene": "UniProtKB:O14804",
  "term_id": "GO:0005886"
}